post-translational protein targeting to membrane, docking [GO:0031203] (biological process) Also known as: Sec-translated protein complex assembly, posttranslational protein membrane targeting, docking, posttranslational protein targeting to membrane, docking, protein docking during posttranslational protein targeting to membrane Definition: The process in which the signal sequence of a translated protein binds to and forms a complex with the Sec complex. References: PMID:12518217, PMID:8707814 Relationships: is a type of protein-containing complex assembly [GO:0065003]; is part of post-translational protein targeting to endoplasmic reticulum membrane [GO:0006620]